{
  "gene_name": "Microfibrillar-associated protein 2",
  "term_label": "embryonic eye morphogenesis",
  "gene_symbol": "MFAP2",
  "gene": "UniProtKB:P55001",
  "term_id": "GO:0048048"
}